phosphatase activity [GO:0016791] (molecular function) Relationships: is a type of phosphoric ester hydrolase activity [GO:0042578] Also known as: phosphoric monoester hydrolase activity, phosphatase Definition: Catalysis of the hydrolysis of a phosphoric monoester, releasing a phosphate. Sources: GOC:curators, GOC:pg Regulation: RO_0002211 by regulation of phosphatase activity [GO:0010921]; positively regulated by positive regulation of phosphatase activity [GO:0010922]; negatively regulated by negative regulation of phosphatase activity [GO:0010923]; regulated by GO:0019208; positively regulated by phosphatase activator activity [GO:0019211]; negatively regulated by GO:0019212 Subtypes: GO:0000121, GO:0002953, GO:0003993, alkaline phosphatase activity [GO:0004035], GO:0004401, polynucleotide 5'-phosphatase activity [GO:0004651], phosphoprotein phosphatase activity [GO:0004721], nucleotidase activity [GO:0008252], phosphatidylglycerophosphatase activity [GO:0008962], phosphoglycolate phosphatase activity [GO:0008967], GO:0019143, GO:0019178, carbohydrate phosphatase activity [GO:0019203], pyridoxal phosphatase activity [GO:0033883], 10-hydroxy-9-(phosphonooxy)octadecanoate phosphatase activity [GO:0033885], D-glycero-beta-D-manno-heptose 1,7-bisphosphate 7-phosphatase activity [GO:0034200], bisphosphoglycerate 3-phosphatase activity [GO:0034417], GO:0036424, thiamine phosphate phosphatase activity [GO:0042131], lipid phosphatase activity [GO:0042577], sn-glycerol 3-phosphatase activity [GO:0043136], 2-hydroxy-3-keto-5-methylthiopentenyl-1-phosphate phosphatase activity [GO:0043716], 5-amino-6-(5-phosphoribitylamino)uracil phosphatase activity [GO:0043726], alpha-ribazole phosphatase activity [GO:0043755], GO:0043874, polynucleotide 3'-phosphatase activity [GO:0046403], methylphosphothioglycerate phosphatase activity [GO:0047382], guanidinodeoxy-scyllo-inositol-4-phosphatase activity [GO:0047383], 2-carboxy-D-arabinitol-1-phosphatase activity [GO:0047538], 3-phosphoglycerate phosphatase activity [GO:0047572], ADP-phosphoglycerate phosphatase activity [GO:0047630], alkylacetylglycerophosphatase activity [GO:0047647], GO:0047846, dolichyl-phosphatase activity [GO:0047873], glycerol-2-phosphatase activity [GO:0047954], mannitol-1-phosphatase activity [GO:0050084], monoterpenyl-diphosphatase activity [GO:0050108], N-acylneuraminate-9-phosphatase activity [GO:0050124], phosphoenolpyruvate phosphatase activity [GO:0050189], phosphoglycerate phosphatase activity [GO:0050192], sedoheptulose-bisphosphatase activity [GO:0050278], sorbitol-6-phosphatase activity [GO:0050286], streptomycin-6-phosphatase activity [GO:0050301], glucosylglycerol 3-phosphatase activity [GO:0050530], mannosyl-3-phosphoglycerate phosphatase activity [GO:0050531], GO:0050532, lysophosphatidic acid phosphatase activity [GO:0052642], GO:0052731, phosphoethanolamine phosphatase activity [GO:0052732], inositol phosphate phosphatase activity [GO:0052745], GO:0052866, dihydrosphingosine-1-phosphate phosphatase activity [GO:0070780], FMN hydrolase activity [GO:0090711], 3',5'-nucleotide bisphosphate phosphatase activity [GO:0097657], ecdysteroid-phosphate phosphatase activity [GO:0102531], NADPH phosphatase activity [GO:0102757], fructose-1-phosphatase activity [GO:0103026], ribitol-5-phosphatase activity [GO:0110130], RNA 2',3'-cyclic phosphatase activity [GO:0160272], GO:0160273, pseudouridine 5'-phosphatase activity [GO:1990738]